mannosyl-inositol phosphorylceramide phospholipase activity [GO:0052714] (molecular function) Sources: GOC:ai Relationships: is a type of GO:0052713 Definition: Catalysis of the reaction: mannosyl-inositol phosphorylceramide + H2O = C26-phytoceramide + mannosylphosphorylinositol.